{
  "term_label": "interleukin-6 receptor activity",
  "term_id": "GO:0004915",
  "gene_symbol": "IL6ST",
  "gene": "UniProtKB:P40189",
  "gene_name": "Interleukin-6 receptor subunit beta"
}